{
  "gene_symbol": "PEBP4",
  "term_label": "Unknown cellular component",
  "gene": "UniProtKB:Q96S96",
  "gene_name": "Phosphatidylethanolamine-binding protein 4",
  "term_id": "UNKNOWN:0003"
}